nitric oxide mediated signal transduction [GO:0007263] (biological process) Subtypes: nitric oxide-cGMP-mediated signaling [GO:0038060] Also known as: NO mediated signal transduction, NO-mediated signal transduction, nitric oxide signaling, nitric oxide-mediated signal transduction Relationships: is a type of intracellular signaling cassette [GO:0141124] Definition: An intracellular signaling cassette that starts with production of nitric oxide, detection by receptors/sensors for nitric oxide (such as soluble guanylyl cyclase/sGC) and ends with the activation of downstream effectors that further transmit the signal within the cell. Nitric oxide transmits its downstream effects through either cyclic GMP (cGMP)-dependent or independent mechanisms. Regulation: regulated by regulation of nitric oxide mediated signal transduction [GO:0010749]; positively regulated by positive regulation of nitric oxide mediated signal transduction [GO:0010750]; negatively regulated by GO:0010751 References: PMID:21549190 Sources: GOC:jl